{
  "gene_name": "Late cornified envelope-like proline-rich protein 1",
  "gene": "UniProtKB:Q5T871",
  "gene_symbol": "LELP1",
  "term_label": "Unknown cellular component",
  "term_id": "UNKNOWN:0003"
}